{
  "term_id": "GO:0046872",
  "term_label": "metal ion binding",
  "gene_name": "Metallothionein 1H-like protein 1",
  "gene": "UniProtKB:P0DM35",
  "gene_symbol": "MT1HL1"
}